{
  "term_id": "UNKNOWN:0001",
  "gene_name": "M-phase-specific PLK1-interacting protein",
  "gene_symbol": "MPLKIP",
  "gene": "UniProtKB:Q8TAP9",
  "term_label": "Unknown molecular function"
}